{
  "term_id": "GO:0042605",
  "gene": "UniProtKB:Q30154",
  "gene_name": "HLA class II histocompatibility antigen, DR beta 5 chain",
  "term_label": "peptide antigen binding",
  "gene_symbol": "HLA-DRB5"
}